{
  "gene_symbol": "RUNX2",
  "gene_name": "Runt-related transcription factor 2",
  "gene": "UniProtKB:Q13950",
  "term_label": "regulation of transcription by RNA polymerase II",
  "term_id": "GO:0006357"
}